{
  "gene_symbol": "PBX4",
  "gene": "UniProtKB:Q9BYU1",
  "term_label": "RNA polymerase II cis-regulatory region sequence-specific DNA binding",
  "gene_name": "Pre-B-cell leukemia transcription factor 4",
  "term_id": "GO:0000978"
}